{
  "term_id": "GO:0031175",
  "term_label": "neuron projection development",
  "gene_name": "Microtubule-associated protein 4",
  "gene": "UniProtKB:P27816",
  "gene_symbol": "MAP4"
}